{
  "term_id": "GO:0030099",
  "term_label": "myeloid cell differentiation",
  "gene_symbol": "CEBPA",
  "gene_name": "CCAAT_enhancer-binding protein alpha",
  "gene": "UniProtKB:P49715"
}